isoleucine biosynthetic process [GO:0009097] (biological process) Definition: The chemical reactions and pathways resulting in the formation of isoleucine, (2R*,3R*)-2-amino-3-methylpentanoic acid. Sources: GOC:ai Also known as: isoleucine anabolism, isoleucine biosynthesis, isoleucine formation, isoleucine synthesis Relationships: is a type of isoleucine metabolic process [GO:0006549]; is a type of branched-chain amino acid biosynthetic process [GO:0009082]; is a type of alpha-amino acid biosynthetic process [GO:1901607] Subtypes: GO:1901705